{
  "gene_symbol": "VAMP1",
  "term_id": "GO:0005484",
  "gene_name": "Vesicle-associated membrane protein 1",
  "gene": "UniProtKB:P23763",
  "term_label": "SNAP receptor activity"
}